2,3-diaminopropionate N-oxalyltransferase activity [GO:0047189] (molecular function) Relationships: is a type of acyltransferase activity, transferring groups other than amino-acyl groups [GO:0016747] Also known as: ODAP synthase activity, oxalyl-CoA:L-2,3-diaminopropanoate 3-N-oxalyltransferase activity, oxalyl-CoA:L-2,3-diaminopropanoate N3-oxalyltransferase activity, oxalyl-CoA:L-alpha,beta-diaminopropionic acid oxalyltransferase activity, oxalyldiaminopropionate synthase activity, oxalyldiaminopropionic synthase activity Sources: RHEA:13465 Definition: Catalysis of the reaction: 3-amino-L-alanine + oxalyl-CoA = N(3)-oxalyl-L-2,3-diaminopropanoate + CoA.